{
  "term_id": "UNKNOWN:0003",
  "gene_name": "DALR anticodon-binding domain-containing protein 3",
  "gene_symbol": "DALRD3",
  "gene": "UniProtKB:Q5D0E6",
  "term_label": "Unknown cellular component"
}